{
  "term_label": "Unknown molecular function",
  "term_id": "UNKNOWN:0001",
  "gene_symbol": "NTS",
  "gene_name": "Neurotensin_neuromedin N",
  "gene": "UniProtKB:P30990"
}